{
  "term_id": "GO:0098839",
  "gene_symbol": "LRFN1",
  "gene": "UniProtKB:Q9P244",
  "term_label": "postsynaptic density membrane",
  "gene_name": "Leucine-rich repeat and fibronectin type III domain-containing protein 1"
}